{
  "term_label": "regulation of transcription by RNA polymerase II",
  "term_id": "GO:0006357",
  "gene_name": "Zinc finger protein ZXDC",
  "gene": "UniProtKB:Q2QGD7",
  "gene_symbol": "ZXDC"
}